{
  "term_id": "UNKNOWN:0003",
  "gene_symbol": "USF3",
  "gene": "UniProtKB:Q68DE3",
  "term_label": "Unknown cellular component",
  "gene_name": "Basic helix-loop-helix domain-containing protein USF3"
}